{
  "gene_name": "Potassium voltage-gated channel subfamily E regulatory beta subunit 5",
  "term_label": "voltage-gated potassium channel complex",
  "gene_symbol": "KCNE5",
  "gene": "UniProtKB:Q9UJ90",
  "term_id": "GO:0008076"
}